{
  "gene_name": "Signal transducer and activator of transcription 6",
  "term_label": "nucleus",
  "gene": "UniProtKB:P42226",
  "term_id": "GO:0005634",
  "gene_symbol": "STAT6"
}